positive regulation of gluconate transmembrane transport [GO:0035432] (biological process) Sources: GOC:vw Definition: Any process that activates or increases the frequency, rate or extent of the directed movement of gluconate across a membrane by means of some agent such as a transporter or pore. Also known as: positive regulation of gluconate membrane transport, up regulation of gluconate transport, up-regulation of gluconate transport, upregulation of gluconate transport, activation of gluconate transport, induction of gluconate transport, stimulation of gluconate transport, positive regulation of gluconate transport Relationships: is a type of positive regulation of organic acid transport [GO:0032892]; is_a positive regulation of transmembrane transport [GO:0034764]; is a type of GO:0035430; positively regulates gluconate transmembrane transport [GO:0035429]